ciliary neurotrophic factor binding [GO:0070119] (molecular function) Sources: GOC:BHF, GOC:mah Relationships: is a type of cytokine binding [GO:0019955] Definition: Binding to the cytokine ciliary neurotrophic factor. Also known as: CNTF binding